positive regulation of MyD88-dependent toll-like receptor signaling pathway [GO:0034126] (biological process) Relationships: is a type of positive regulation of toll-like receptor signaling pathway [GO:0034123]; is a type of regulation of MyD88-dependent toll-like receptor signaling pathway [GO:0034124]; positively regulates MyD88-dependent toll-like receptor signaling pathway [GO:0002755] Also known as: positive regulation of MyD88-dependent TLR signaling pathway, positive regulation of MyD88-dependent toll-like receptor signalling pathway References: PMID:16551253, PMID:17328678 Sources: GOC:add Definition: Any process that activates or increases the frequency, rate, or extent of MyD88-dependent toll-like receptor signaling pathway.